{
  "term_id": "GO:0035371",
  "gene_name": "Microtubule-associated protein RP_EB family member 1",
  "gene_symbol": "MAPRE1",
  "gene": "UniProtKB:Q15691",
  "term_label": "microtubule plus-end"
}